positive regulation of Golgi lumen acidification [GO:1905528] (biological process) Definition: Any process that activates or increases the frequency, rate or extent of Golgi lumen acidification. Relationships: is a type of positive regulation of cellular pH reduction [GO:0032849]; is a type of regulation of Golgi lumen acidification [GO:1905526]; positively regulates Golgi lumen acidification [GO:0061795] References: PMID:23447592 Sources: GOC:TermGenie, GOC:dph, GO_REF:0000058 Also known as: up regulation of Golgi lumen acidification, up-regulation of Golgi lumen acidification, upregulation of Golgi lumen acidification, activation of Golgi lumen acidification